regulation of vesicle size [GO:0097494] (BP) Definition: Any process that modulates the size of a vesicle. Subtypes: regulation of post-lysosomal vacuole size [GO:0044656], GO:0051036 References: PMID:20007772 Sources: GOC:pm Relationships: is_a regulation of cellular component size [GO:0032535]